{
  "term_id": "UNKNOWN:0001",
  "gene_symbol": "SKAP1",
  "gene_name": "Src kinase-associated phosphoprotein 1",
  "gene": "UniProtKB:Q86WV1",
  "term_label": "Unknown molecular function"
}